{
  "gene_symbol": "WDR54",
  "gene": "UniProtKB:Q9H977",
  "term_id": "GO:0031514",
  "gene_name": "WD repeat-containing protein 54",
  "term_label": "motile cilium"
}